{
  "gene_name": "Ubiquitin-conjugating enzyme E2 G2",
  "gene": "UniProtKB:P60604",
  "term_id": "GO:0006511",
  "term_label": "ubiquitin-dependent protein catabolic process",
  "gene_symbol": "UBE2G2"
}